{
  "term_label": "structural constituent of nuclear pore",
  "gene_name": "Nuclear pore complex protein Nup153",
  "term_id": "GO:0017056",
  "gene": "UniProtKB:P49790",
  "gene_symbol": "NUP153"
}